{
  "gene": "UniProtKB:A0N4X2",
  "gene_name": "Possible J 40 gene segment (Fragment)",
  "term_label": "Unknown biological process",
  "gene_symbol": "TRAJ40",
  "term_id": "UNKNOWN:0002"
}